kaempferide 7-O-methyltransferase activity [GO:0102450] (molecular function) Relationships: is a type of GO:0008168 Definition: Catalysis of the reaction: kaempferide + S-adenosyl-L-methionine = 7,4'-O-dimethylkaempferol + H+ + S-adenosyl-L-homocysteine. Sources: RHEA:74775